{
  "gene": "UniProtKB:Q7RTS5",
  "term_id": "GO:0042802",
  "gene_name": "Proton channel OTOP3",
  "gene_symbol": "OTOP3",
  "term_label": "identical protein binding"
}